{
  "term_label": "nucleus",
  "gene_symbol": "MSH4",
  "gene_name": "MutS protein homolog 4",
  "gene": "UniProtKB:O15457",
  "term_id": "GO:0005634"
}